{
  "gene_name": "Transmembrane protein 82",
  "gene_symbol": "TMEM82",
  "term_label": "Unknown molecular function",
  "gene": "UniProtKB:A0PJX8",
  "term_id": "UNKNOWN:0001"
}